{
  "gene": "UniProtKB:A6PVI3",
  "gene_symbol": "NCBP2L",
  "gene_name": "Nuclear cap-binding protein subunit 2-like",
  "term_label": "mRNA splicing, via spliceosome",
  "term_id": "GO:0000398"
}